regulation of potassium ion transmembrane transport [GO:1901379] (biological process) Subtypes: GO:1901380, positive regulation of potassium ion transmembrane transport [GO:1901381], regulation of potassium ion import [GO:1903286], GO:1903764 Sources: GOC:BHF, GOC:TermGenie Also known as: regulation of potassium ion membrane transport Relationships: is a type of regulation of potassium ion transport [GO:0043266]; is a type of regulation of monoatomic cation transmembrane transport [GO:1904062]; regulates potassium ion transmembrane transport [GO:0071805] Definition: Any process that modulates the frequency, rate or extent of potassium ion transmembrane transport.